{
  "term_id": "UNKNOWN:0001",
  "gene_name": "Glioma pathogenesis-related protein 1",
  "gene_symbol": "GLIPR1",
  "term_label": "Unknown molecular function",
  "gene": "UniProtKB:P48060"
}